{
  "term_label": "regulation of neuronal synaptic plasticity",
  "gene": "UniProtKB:Q13555",
  "term_id": "GO:0048168",
  "gene_symbol": "CAMK2G",
  "gene_name": "Calcium_calmodulin-dependent protein kinase type II subunit gamma"
}